{
  "gene_symbol": "TMPRSS6",
  "gene": "UniProtKB:Q8IU80",
  "term_id": "GO:0016485",
  "term_label": "protein processing",
  "gene_name": "Transmembrane protease serine 6"
}